{
  "gene_name": "Importin-7",
  "term_id": "GO:0061608",
  "gene_symbol": "IPO7",
  "gene": "UniProtKB:O95373",
  "term_label": "nuclear import signal receptor activity"
}